{
  "gene_symbol": "CNGA2",
  "gene_name": "Cyclic nucleotide-gated olfactory channel",
  "term_id": "GO:0030553",
  "term_label": "cGMP binding",
  "gene": "UniProtKB:Q16280"
}